{
  "term_label": "plasma membrane",
  "term_id": "GO:0005886",
  "gene_symbol": "CR2",
  "gene": "UniProtKB:P20023",
  "gene_name": "Complement receptor type 2"
}